{
  "term_label": "DNA-binding transcription factor activity, RNA polymerase II-specific",
  "gene_symbol": "HES6",
  "term_id": "GO:0000981",
  "gene": "UniProtKB:Q96HZ4",
  "gene_name": "Transcription cofactor HES-6"
}